{
  "gene_symbol": "SIRT1",
  "term_id": "GO:0005654",
  "gene": "UniProtKB:Q96EB6",
  "gene_name": "NAD-dependent protein deacetylase sirtuin-1",
  "term_label": "nucleoplasm"
}